negative regulation of connective tissue growth factor production [GO:0032683] (biological process) Also known as: down regulation of connective tissue growth factor production, down-regulation of connective tissue growth factor production, downregulation of connective tissue growth factor production, negative regulation of CCN2 production, negative regulation of CTGF production, negative regulation of Fisp12 production, negative regulation of Hcs24 production, negative regulation of IGFBP8 production, negative regulation of hypertrophic chondrocyte-specific gene product 24 production, inhibition of connective tissue growth factor production, negative regulation of connective tissue growth factor biosynthetic process Definition: Any process that stops, prevents, or reduces the frequency, rate, or extent of connective tissue growth factor production. Sources: GOC:mah Relationships: is a type of negative regulation of cytokine production [GO:0001818]; is a type of regulation of connective tissue growth factor production [GO:0032643]; negatively regulates GO:0032601